{
  "gene_name": "Hyaluronidase-3",
  "gene_symbol": "HYAL3",
  "term_label": "hyaluronan catabolic process",
  "term_id": "GO:0030214",
  "gene": "UniProtKB:O43820"
}